{
  "gene_symbol": "SOHLH1",
  "term_label": "Unknown biological process",
  "term_id": "UNKNOWN:0002",
  "gene_name": "Spermatogenesis- and oogenesis-specific basic helix-loop-helix-containing protein 1",
  "gene": "UniProtKB:Q5JUK2"
}